histone H3K27 dimethyltransferase activity [GO:0140952] (molecular function) Definition: Catalysis of the reaction: L-lysyl27-[histone H3] + 2 S-adenosyl-L-methionine = 2 H+ + N6,N6-dimethyl-L-lysyl27-[histone H3] + 2 S-adenosyl-L-homocysteine. This reaction is the successive addition of two methyl groups to the unmethylated lysine residue at position 27 of histone H3, producing histone H3K27me2. Sources: RHEA:64452 Also known as: histone H3-K27 dimethylation, histone H3K27 dimethylation, histone H3-K27 dimethylase activity, histone H3K27 dimethylase activity, histone H3K27 mono/dimethylase activity, histone lysine N-dimethyltransferase activity (H3-K27 specific) Note: Comment: Note that the residue position corresponds to the canonical human H3 histone (UniProtKB:P84243); this residue is conserved across all eukaryotes. Residue 1 is the first residue following removal of the initiating Methionine (Met). Note that each histone is encoded by multiple genes, and sequences may vary across different genes within an organism. Relationships: is_a histone H3K27 methyltransferase activity [GO:0046976]